{
  "gene_symbol": "GNG8",
  "gene": "UniProtKB:Q9UK08",
  "term_label": "G protein-coupled receptor signaling pathway",
  "term_id": "GO:0007186",
  "gene_name": "Guanine nucleotide-binding protein G(I)_G(S)_G(O) subunit gamma-8"
}